iduronate-2-sulfatase activity [GO:0004423] (molecular function) Also known as: chondroitinsulfatase, iduronate-2-sulphatase activity, 2-sulfo-L-iduronate 2-sulfatase activity, L-iduronate 2-sulfate sulfatase activity, L-iduronate-2-sulfate 2-sulfohydrolase activity, L-idurono sulfate sulfatase activity, L-iduronosulfatase activity, iduronate sulfatase activity, iduronate sulfate sulfatase activity, iduronate-2-sulfate sulfatase activity, iduronide-2-sulfate sulfatase activity, idurono-2-sulfatase activity, sulfo-L-iduronate sulfatase activity, sulfoiduronate sulfohydrolase activity Relationships: is a type of sulfuric ester hydrolase activity [GO:0008484] Sources: EC:3.1.6.13 Definition: Catalysis of the hydrolysis of the 2-sulfate groups of the L-iduronate 2-sulfate units of dermatan sulfate, heparan sulfate and heparin.